{
  "term_label": "positive regulation of actin filament bundle assembly",
  "term_id": "GO:0032233",
  "gene_symbol": "SYNPO",
  "gene_name": "Synaptopodin",
  "gene": "UniProtKB:Q8N3V7"
}